{
  "gene": "UniProtKB:Q8N4Q0",
  "term_label": "15-oxoprostaglandin 13-reductase [NAD(P)+] activity",
  "term_id": "GO:0047522",
  "gene_symbol": "PTGR3",
  "gene_name": "Prostaglandin reductase 3"
}